{
  "gene": "UniProtKB:Q9NUB1",
  "gene_symbol": "ACSS1",
  "term_id": "GO:0006085",
  "gene_name": "Acetyl-coenzyme A synthetase 2-like, mitochondrial",
  "term_label": "acetyl-CoA biosynthetic process"
}